{
  "gene_symbol": "TTC4",
  "gene_name": "Tetratricopeptide repeat protein 4",
  "term_label": "Hsp70 protein binding",
  "gene": "UniProtKB:O95801",
  "term_id": "GO:0030544"
}